regulation of androgen receptor signaling pathway [GO:0060765] (biological process) Definition: Any process that modulates the rate, frequency, or extent of the androgen receptor signaling pathway. Sources: GOC:dph Subtypes: negative regulation of androgen receptor signaling pathway [GO:0060766], positive regulation of androgen receptor signaling pathway [GO:0160207] Relationships: is a type of GO:0033143; regulates androgen receptor signaling pathway [GO:0030521] Also known as: regulation of androgen receptor signalling pathway